{
  "gene": "UniProtKB:Q13324",
  "gene_symbol": "CRHR2",
  "gene_name": "Corticotropin-releasing factor receptor 2",
  "term_id": "GO:0043404",
  "term_label": "corticotropin-releasing hormone receptor activity"
}